{
  "gene_name": "HERV-H LTR-associating protein 1",
  "term_label": "Unknown cellular component",
  "term_id": "UNKNOWN:0003",
  "gene_symbol": "HHLA1",
  "gene": "UniProtKB:C9JL84"
}